{
  "term_label": "membrane",
  "gene": "UniProtKB:Q8NFQ8",
  "gene_name": "Torsin-1A-interacting protein 2",
  "term_id": "GO:0016020",
  "gene_symbol": "TOR1AIP2"
}